{
  "term_id": "GO:0045824",
  "gene_name": "Splicing factor Cactin",
  "gene": "UniProtKB:Q8WUQ7",
  "gene_symbol": "CACTIN",
  "term_label": "negative regulation of innate immune response"
}